mannan 1,2-(1,3)-alpha-mannosidase activity [GO:0033915] (molecular function) Definition: Catalysis of the hydrolysis of (1->2) and (1->3) linkages in mannan, releasing mannose. Sources: EC:3.2.1.77 Also known as: 1,2-1,3-alpha-D-mannan mannohydrolase activity, exo-1,2-1,3-alpha-mannosidase activity Relationships: is a type of alpha-mannosidase activity [GO:0004559]